{
  "gene_name": "Inactive serine_threonine-protein kinase TEX14",
  "term_id": "GO:0007140",
  "gene": "UniProtKB:Q8IWB6",
  "term_label": "male meiotic nuclear division",
  "gene_symbol": "TEX14"
}